purine nucleotide salvage [GO:0032261] (biological process) Definition: Any process which produces a purine nucleotide from derivatives of it, without de novo synthesis. Relationships: is a type of purine nucleotide biosynthetic process [GO:0006164]; is a type of purine-containing compound salvage [GO:0043101]; is a type of nucleotide salvage [GO:0043173] Subtypes: GO:0034355, purine ribonucleotide salvage [GO:0106380], purine deoxyribonucleotide salvage [GO:0106381] Sources: GOC:jp